{
  "term_label": "establishment or maintenance of cell polarity",
  "term_id": "GO:0007163",
  "gene_symbol": "ANKRD6",
  "gene_name": "Ankyrin repeat domain-containing protein 6",
  "gene": "UniProtKB:Q9Y2G4"
}